5'-3' RNA exonuclease activity [GO:0004534] (molecular function) Definition: Catalysis of the sequential cleavage of mononucleotides from a free 5' terminus of an RNA molecule. Sources: GOC:mah, ISBN:0198547684 Also known as: 5'-3' exoribonuclease activity Relationships: is a type of GO:0008409; is_a GO:0016896